regulation of phosphatidylethanolamine metabolic process [GO:0150175] (biological process) References: PMID:30074985 Sources: GOC:aruk, GOC:bc Relationships: is a type of GO:1903725; regulates phosphatidylethanolamine metabolic process [GO:0046337] Definition: Any process that modulates the frequency, rate or extent of phosphatidylethanolamine metabolic process.